{
  "term_label": "Unknown biological process",
  "term_id": "UNKNOWN:0002",
  "gene_name": "Protein bicaudal C homolog 1",
  "gene": "UniProtKB:Q9H694",
  "gene_symbol": "BICC1"
}